{
  "term_id": "GO:0043235",
  "gene": "UniProtKB:Q9UJ42",
  "term_label": "receptor complex",
  "gene_symbol": "GPR160",
  "gene_name": "Probable G-protein coupled receptor 160"
}